{
  "term_label": "chromatin binding",
  "gene_symbol": "CBX8",
  "gene": "UniProtKB:Q9HC52",
  "term_id": "GO:0003682",
  "gene_name": "Chromobox protein homolog 8"
}